venom-mediated perturbation of voltage-gated potassium channel activity [GO:0044559] (biological process) Also known as: envenomation resulting in modulation of voltage-gated potassium channel activity in another organism, envenomation resulting in modulation of voltage-gated potassium channel activity in other organism Subtypes: venom-mediated inhibition of voltage-gated potassium channel activity [GO:0044562] Definition: A process in which an organism alters or subverts the activity of a voltage-gated potassium channel in another organism via the action of a venom. Relationships: is a type of venom-mediated perturbation of ion channel activity [GO:0044560] Sources: GOC:fj, GOC:jl